{
  "term_label": "microtubule",
  "gene_name": "Kinesin-like protein KIF15",
  "term_id": "GO:0005874",
  "gene": "UniProtKB:Q9NS87",
  "gene_symbol": "KIF15"
}